hydroxymethylglutaryl-CoA hydrolase activity [GO:0047994] (molecular function) Sources: EC:3.1.2.5, RHEA:16305 Relationships: is a type of acyl-CoA hydrolase activity [GO:0016289] Definition: Catalysis of the reaction: (S)-3-hydroxy-3-methylglutaryl-CoA + H2O = 3-hydroxy-3-methylglutarate + CoA + H+. Also known as: (S)-3-hydroxy-3-methylglutaryl-CoA hydrolase activity, 3-hydroxy-3-methylglutaryl-CoA hydrolase activity, beta-hydroxy-beta-methylglutaryl coenzyme A deacylase activity, beta-hydroxy-beta-methylglutaryl coenzyme A hydrolase activity, hydroxymethylglutaryl coenzyme A deacylase activity, hydroxymethylglutaryl coenzyme A hydrolase activity